{
  "gene_name": "Histone H3.3C",
  "gene_symbol": "H3-5",
  "gene": "UniProtKB:Q6NXT2",
  "term_label": "kinetochore assembly",
  "term_id": "GO:0051382"
}